putrescine binding [GO:0019810] (molecular function) Definition: Binding to putrescine, 1,4-diaminobutane, the polyamine formed by decarboxylation of ornithine and the metabolic precursor of spermidine and spermine. Relationships: is a type of GO:0019808; is a type of cation binding [GO:0043169] Sources: GOC:ai